steryl deacetylase activity [GO:0034084] (molecular function) References: PMID:18034159 Sources: GOC:rb Also known as: sterol deacetylase activity, steryl acetyl hydrolase activity Definition: Catalysis of the hydrolysis of an acetyl group or groups from an acetylated sterol. Relationships: is a type of hydrolase activity [GO:0016787]; is_a GO:0019213